quinate 3-dehydrogenase (NADP+) activity [GO:0052733] (molecular function) Definition: Catalysis of the reaction: quinate + NADP+ = 3-dehydroquinate + NADPH + H+. Also known as: quinic dehydrogenase activity, quinate:NADP 3-oxidoreductase activity, quinate:NADP(+) 3-oxidoreductase activity Relationships: is a type of GO:0016616 Sources: RHEA:18425